{
  "gene_name": "Serine_threonine-protein kinase PAK 5",
  "gene": "UniProtKB:Q9P286",
  "term_id": "GO:0009267",
  "gene_symbol": "PAK5",
  "term_label": "cellular response to starvation"
}